negative regulation of nucleobase-containing compound metabolic process [GO:0045934] (biological process) Sources: GOC:go_curators Definition: Any cellular process that stops, prevents, or reduces the frequency, rate or extent of the chemical reactions and pathways involving nucleobases, nucleosides, nucleotides and nucleic acids. Also known as: down regulation of nucleobase, nucleoside, nucleotide and nucleic acid metabolic process, down-regulation of nucleobase, nucleoside, nucleotide and nucleic acid metabolic process, downregulation of nucleobase, nucleoside, nucleotide and nucleic acid metabolic process, negative regulation of nucleobase, nucleoside, nucleotide and nucleic acid metabolism, inhibition of nucleobase, nucleoside, nucleotide and nucleic acid metabolic process, negative regulation of nucleobase, nucleoside, nucleotide and nucleic acid metabolic process Subtypes: negative regulation of nucleoside metabolic process [GO:0045978], negative regulation of nucleotide metabolic process [GO:0045980], negative regulation of purine nucleobase metabolic process [GO:0045982], GO:0045984, GO:0051053, GO:0051253, GO:0106279, negative regulation of pyruvate decarboxylation to acetyl-CoA [GO:0160218], negative regulation of butyryl-CoA biosynthetic process from acetyl-CoA [GO:1900495], negative regulation of butyryl-CoA catabolic process to butanol [GO:1900498], GO:1900501, negative regulation of tetrapyrrole biosynthetic process from glycine and succinyl-CoA [GO:1901414], negative regulation of isopentenyl diphosphate biosynthetic process, mevalonate pathway [GO:2001211] Relationships: is a type of negative regulation of metabolic process [GO:0009892]; is a type of regulation of nucleobase-containing compound metabolic process [GO:0019219]; negatively regulates nucleobase-containing compound metabolic process [GO:0006139]